{
  "gene_name": "Thyroxine 5-deiodinase",
  "term_id": "GO:0004800",
  "gene_symbol": "DIO3",
  "gene": "UniProtKB:P55073",
  "term_label": "thyroxine 5'-deiodinase activity"
}